equatorial cell cortex [GO:1990753] (cellular component) Relationships: is a type of cell cortex region [GO:0099738]; is part of cell division site [GO:0032153] References: PMID:16352658, PMID:22552143, PMID:23750214, PMID:25898168 Sources: GOC:kmv Definition: The region of the cell cortex in a mitotically dividing cell that flanks the central spindle and corresponds to the site of actomyosin ring formation that results in cleavage furrow formation and ingression.